{
  "gene_symbol": "CMAHP",
  "gene_name": "Inactive cytidine monophosphate-N-acetylneuraminic acid hydroxylase",
  "term_label": "cytoplasm",
  "gene": "UniProtKB:Q9Y471",
  "term_id": "GO:0005737"
}